{
  "gene_symbol": "OR1B1",
  "gene_name": "Olfactory receptor 1B1",
  "term_label": "olfactory receptor activity",
  "term_id": "GO:0004984",
  "gene": "UniProtKB:Q8NGR6"
}